{
  "gene": "UniProtKB:Q96NS1",
  "term_label": "Unknown cellular component",
  "term_id": "UNKNOWN:0003",
  "gene_symbol": "YPEL4",
  "gene_name": "Protein yippee-like 4"
}